{
  "gene_symbol": "OR10H4",
  "gene": "UniProtKB:Q8NGA5",
  "gene_name": "Olfactory receptor 10H4",
  "term_id": "GO:0050911",
  "term_label": "detection of chemical stimulus involved in sensory perception of smell"
}